U2 snRNA binding [GO:0030620] (molecular function) Sources: GOC:jl Relationships: is a type of snRNA binding [GO:0017069] Definition: Binding to a U2 small nuclear RNA (U2 snRNA).